{
  "gene_name": "Septin-10",
  "term_label": "molecular adaptor activity",
  "term_id": "GO:0060090",
  "gene": "UniProtKB:Q9P0V9",
  "gene_symbol": "SEPTIN10"
}